{
  "gene_symbol": "OSTN",
  "gene": "UniProtKB:P61366",
  "gene_name": "Osteocrin",
  "term_id": "GO:0009755",
  "term_label": "hormone-mediated signaling pathway"
}